{
  "term_label": "Unknown biological process",
  "gene_symbol": "SHANK2-AS3",
  "term_id": "UNKNOWN:0002",
  "gene_name": "Putative uncharacterized protein SHANK2-AS3",
  "gene": "UniProtKB:Q9BTD1"
}